{
  "term_label": "membrane",
  "gene_symbol": "SERINC1",
  "term_id": "GO:0016020",
  "gene": "UniProtKB:Q9NRX5",
  "gene_name": "Serine incorporator 1"
}